{
  "gene_name": "X antigen family member 1",
  "gene": "UniProtKB:Q9HD64",
  "gene_symbol": "XAGE1B",
  "term_id": "UNKNOWN:0001",
  "term_label": "Unknown molecular function"
}